{
  "term_id": "GO:0031201",
  "gene_name": "Syntaxin-19",
  "gene_symbol": "STX19",
  "term_label": "SNARE complex",
  "gene": "UniProtKB:Q8N4C7"
}